{
  "term_label": "Unknown molecular function",
  "gene": "UniProtKB:Q6SZW1",
  "gene_name": "NAD(+) hydrolase SARM1",
  "gene_symbol": "SARM1",
  "term_id": "UNKNOWN:0001"
}